{
  "term_id": "GO:0030139",
  "gene": "UniProtKB:P14317",
  "gene_symbol": "HCLS1",
  "gene_name": "Hematopoietic lineage cell-specific protein",
  "term_label": "endocytic vesicle"
}